negative regulation of icosanoid secretion [GO:0032304] (biological process) Definition: Any process that stops, prevents, or reduces the frequency, rate or extent of the controlled release of an icosanoid from a cell. Also known as: down regulation of icosanoid secretion, down-regulation of icosanoid secretion, downregulation of icosanoid secretion, negative regulation of eicosanoid secretion, inhibition of icosanoid secretion Subtypes: negative regulation of prostaglandin secretion [GO:0032307], negative regulation of arachidonate secretion [GO:1900139] Sources: GOC:mah Relationships: is a type of GO:0032303; is a type of negative regulation of secretion [GO:0051048]; is a type of negative regulation of fatty acid transport [GO:2000192]; negatively regulates GO:0032309